{
  "gene_symbol": "FNTA",
  "gene": "UniProtKB:P49354",
  "term_id": "GO:0007323",
  "gene_name": "Protein farnesyltransferase_geranylgeranyltransferase type-1 subunit alpha",
  "term_label": "peptide pheromone maturation"
}